{
  "term_id": "GO:0005347",
  "gene": "UniProtKB:Q8N5S1",
  "term_label": "ATP transmembrane transporter activity",
  "gene_symbol": "SLC25A41",
  "gene_name": "Mitochondrial carrier protein SCaMC-3L"
}